rRNA binding [GO:0019843] (molecular function) Relationships: is a type of RNA binding [GO:0003723] Subtypes: 5S rRNA binding [GO:0008097], GO:0030556, rRNA primary transcript binding [GO:0042134], large ribosomal subunit rRNA binding [GO:0070180], small ribosomal subunit rRNA binding [GO:0070181], 5.8S rRNA binding [GO:1990932] Sources: GOC:jl Definition: Binding to a ribosomal RNA. Also known as: base pairing with rRNA